{
  "term_id": "GO:0000165",
  "term_label": "MAPK cascade",
  "gene_symbol": "MINK1",
  "gene": "UniProtKB:Q8N4C8",
  "gene_name": "Misshapen-like kinase 1"
}